{
  "gene_symbol": "SHANK3",
  "gene": "UniProtKB:Q9BYB0",
  "gene_name": "SH3 and multiple ankyrin repeat domains protein 3",
  "term_label": "postsynaptic density",
  "term_id": "GO:0014069"
}